response to low fluence blue light stimulus by blue low-fluence system [GO:0010244] (biological process) Definition: Any process that results in a change in state or activity of a cell or an organism (in terms of movement, secretion, enzyme production, gene expression, etc.) as a result of the detection of a low fluence blue light stimulus by the blue low-fluence system. Blue light is electromagnetic radiation with a wavelength of between 440 and 500nm. The blue low-fluence system responds to blue light at or below 0.1 micromols/m2. In certain species excitation of the blue low fluence system induces the transcription of a number of nuclear and plastid coded genes. Relationships: is a type of response to blue light [GO:0009637]; is a type of response to low light intensity stimulus [GO:0009645] Also known as: response to low fluence blue light, response to low fluence blue light by blf system References: PMID:10398709 Sources: GOC:mtg_far_red